{
  "gene_name": "Tax1-binding protein 3",
  "gene_symbol": "TAX1BP3",
  "term_id": "UNKNOWN:0002",
  "term_label": "Unknown biological process",
  "gene": "UniProtKB:O14907"
}